4-hydroxybenzoate polyprenyltransferase activity [GO:0008412] (molecular function) Relationships: is a type of prenyltransferase activity [GO:0004659] Sources: RHEA:44504 Definition: Catalysis of the reaction: 4-hydroxybenzoate + an all-trans-polyprenyl diphosphate = a 4-hydroxy-3-all-trans-polyprenylbenzoate + diphosphate. Also known as: 4-HB polyprenyltransferase activity, PHB polyprenyl diphosphate transferase activity, para-hydroxybenzoate transferase activity, para-hydroxybenzoate-polyprenyl diphosphate transferase activity, para-hydroxybenzoate:polyprenyltransferase activity, 4-hydroxybenzoate nonaprenyltransferase activity